{
  "gene_symbol": "TSPAN19",
  "term_label": "Unknown molecular function",
  "gene": "UniProtKB:P0C672",
  "term_id": "UNKNOWN:0001",
  "gene_name": "Tetraspanin-19"
}